{
  "gene_symbol": "CYFIP2",
  "term_id": "UNKNOWN:0001",
  "gene_name": "Cytoplasmic FMR1-interacting protein 2",
  "gene": "UniProtKB:Q96F07",
  "term_label": "Unknown molecular function"
}